regulation of immune response to tumor cell [GO:0002837] (biological process) Also known as: regulation of immune response to tumour cell Sources: GOC:add Definition: Any process that modulates the frequency, rate, or extent of an immune response to tumor cell. Relationships: is a type of regulation of response to tumor cell [GO:0002834]; is a type of regulation of immune response [GO:0050776]; regulates immune response to tumor cell [GO:0002418] Subtypes: negative regulation of immune response to tumor cell [GO:0002838], positive regulation of immune response to tumor cell [GO:0002839], regulation of T cell mediated immune response to tumor cell [GO:0002840], GO:0002843, regulation of natural killer cell mediated immune response to tumor cell [GO:0002855]